{
  "term_id": "UNKNOWN:0001",
  "gene_symbol": "JPH3",
  "gene_name": "Junctophilin-3",
  "gene": "UniProtKB:Q8WXH2",
  "term_label": "Unknown molecular function"
}